retinal cone cell fate determination [GO:0042671] (biological process) Relationships: is_a photoreceptor cell fate determination [GO:0043703]; is part of retinal cone cell fate commitment [GO:0046551] Sources: GOC:go_curators Definition: The process in which a cell becomes capable of differentiating autonomously into a retinal cone cell regardless of its environment; upon determination, the cell fate cannot be reversed.